{
  "gene": "UniProtKB:Q9UBI4",
  "term_label": "Unknown biological process",
  "term_id": "UNKNOWN:0002",
  "gene_name": "Stomatin-like protein 1",
  "gene_symbol": "STOML1"
}